{
  "gene_symbol": "AGRN",
  "term_label": "nervous system development",
  "gene": "UniProtKB:O00468",
  "gene_name": "Agrin",
  "term_id": "GO:0007399"
}